{
  "term_id": "GO:0005737",
  "gene": "UniProtKB:P61978",
  "gene_name": "Heterogeneous nuclear ribonucleoprotein K",
  "term_label": "cytoplasm",
  "gene_symbol": "HNRNPK"
}